{
  "gene_symbol": "ST6GALNAC6",
  "term_id": "UNKNOWN:0003",
  "gene": "UniProtKB:Q969X2",
  "term_label": "Unknown cellular component",
  "gene_name": "Alpha-N-acetylgalactosaminide alpha-2,6-sialyltransferase 6"
}